{
  "gene_symbol": "DUS3L",
  "term_label": "Unknown cellular component",
  "term_id": "UNKNOWN:0003",
  "gene": "UniProtKB:Q96G46",
  "gene_name": "tRNA-dihydrouridine(47) synthase [NAD(P)(+)]-like"
}